{
  "term_label": "negative regulation of microglial cell activation",
  "gene_symbol": "CST7",
  "term_id": "GO:1903979",
  "gene": "UniProtKB:O76096",
  "gene_name": "Cystatin-F"
}